short-chain fatty acyl-CoA hydrolase activity [GO:0141126] (molecular function) Definition: Catalysis of the reaction: a short-chain fatty acyl-CoA + H2O = a short fatty acid + CoA + H+. A short-chain fatty acid has an aliphatic tail of less than 6 carbons. Subtypes: 3-hydroxyisobutyryl-CoA hydrolase activity [GO:0003860] Note: While there is not universal consensus on the lengths of short-, medium-, long- and very-long-chain fatty acids, the GO uses the definitions in ChEBI (see CHEBI:26666, CHEBI:59554, CHEBI:15904 and CHEBI:27283). Relationships: is a type of GO:0047617 Sources: RHEA:68180